oxidoreductase activity, acting on the aldehyde or oxo group of donors, cytochrome as acceptor [GO:0016622] (molecular function) Definition: Catalysis of an oxidation-reduction (redox) reaction in which an aldehyde or ketone (oxo) group acts as a hydrogen or electron donor and reduces a cytochrome. Sources: GOC:jl Relationships: is a type of oxidoreductase activity, acting on the aldehyde or oxo group of donors [GO:0016903] Subtypes: GO:0008805, GO:0047111, GO:0047898